{
  "gene": "UniProtKB:Q5W0Z9",
  "gene_name": "Palmitoyltransferase ZDHHC20",
  "term_id": "GO:0006612",
  "gene_symbol": "ZDHHC20",
  "term_label": "protein targeting to membrane"
}